{
  "gene_symbol": "HINT1",
  "gene": "UniProtKB:P49773",
  "term_id": "GO:0005737",
  "gene_name": "Adenosine 5'-monophosphoramidase HINT1",
  "term_label": "cytoplasm"
}